trypanothione-disulfide reductase (NADPH) activity [GO:0015042] (molecular function) Also known as: trypanothione reductase activity, trypanothione-disulfide reductase activity, trypanothione-disulphide reductase activity, NADPH:trypanothione oxidoreductase activity, trypanothione-disulfide reductase (NADP) activity, trypanothione:NADP+ oxidoreductase activity Sources: RHEA:16757 Relationships: is a type of GO:0015036; is a type of GO:0016668 Definition: Catalysis of the reaction: NADP+ + trypanothione = NADPH + H+ + trypanothione disulfide.